{
  "term_id": "GO:0005764",
  "term_label": "lysosome",
  "gene": "UniProtKB:Q9H3U5",
  "gene_name": "Major facilitator superfamily domain-containing protein 1",
  "gene_symbol": "MFSD1"
}